{
  "gene_name": "Frizzled-6",
  "term_label": "non-canonical Wnt signaling pathway",
  "gene": "UniProtKB:O60353",
  "gene_symbol": "FZD6",
  "term_id": "GO:0035567"
}